{
  "term_id": "GO:0008442",
  "gene_name": "3-hydroxyisobutyrate dehydrogenase, mitochondrial",
  "gene": "UniProtKB:P31937",
  "gene_symbol": "HIBADH",
  "term_label": "3-hydroxyisobutyrate dehydrogenase activity"
}